{
  "gene_symbol": "PURG",
  "gene_name": "Purine-rich element-binding protein gamma",
  "term_label": "DNA-binding transcription factor activity, RNA polymerase II-specific",
  "term_id": "GO:0000981",
  "gene": "UniProtKB:Q9UJV8"
}